metanephric glomerular mesangial cell development [GO:0072255] (BP) Definition: The process whose specific outcome is the progression of a glomerular mesangial cell in the metanephros over time, from its formation to the mature structure. Relationships: is_a glomerular mesangial cell development [GO:0072144]; is part of GO:0072254 Sources: GOC:mtg_kidney_jan10